{
  "gene_symbol": "OR8G1",
  "term_id": "GO:0007186",
  "gene_name": "Olfactory receptor 8G1",
  "gene": "UniProtKB:Q15617",
  "term_label": "G protein-coupled receptor signaling pathway"
}